regulation of meiosis I [GO:0060631] (biological process) Relationships: is a type of regulation of meiotic nuclear division [GO:0040020]; regulates meiosis I [GO:0007127] Sources: GOC:dph, GOC:tb Subtypes: GO:0060903, GO:0110029, regulation of meiosis I spindle assembly checkpoint [GO:1905325] Definition: Any process that modulates the rate, frequency, or extent of meiosis I, a cell cycle process comprising the steps by which a cell progresses through the first phase of meiosis, in which cells divide and homologous chromosomes are paired and segregated from each other, producing two daughter cells.